Nem1-Spo7 phosphatase complex [GO:0071595] (cellular component) References: PMID:9822591 Sources: GOC:mah Relationships: is_a protein serine/threonine phosphatase complex [GO:0008287]; is a type of GO:0098796; is part of nuclear outer membrane-endoplasmic reticulum membrane network [GO:0042175] Definition: A protein serine/threonine phosphatase complex that is involved in nuclear envelope organization, and contains proteins known in budding yeast as Nem1p and Spo7p.